{
  "term_id": "UNKNOWN:0001",
  "gene": "UniProtKB:Q8NE31",
  "gene_name": "Protein FAM13C",
  "term_label": "Unknown molecular function",
  "gene_symbol": "FAM13C"
}